vesicle targeting, trans-Golgi to endosome [GO:0048203] (biological process) Definition: The process in which vesicles are directed to specific destination membranes during transport from the trans-Golgi to the endosome. Relationships: is a type of vesicle targeting, to, from or within Golgi [GO:0048199]; BFO_0000050 Golgi to endosome transport [GO:0006895] References: PMID:10219233 Sources: GOC:jid, GOC:mah, ISBN:0716731363 Also known as: trans-Golgi to endosome targeting